{
  "gene_name": "Adenomatous polyposis coli protein",
  "gene": "UniProtKB:P25054",
  "gene_symbol": "APC",
  "term_id": "GO:0016477",
  "term_label": "cell migration"
}